{
  "term_id": "GO:0017128",
  "term_label": "phospholipid scramblase activity",
  "gene": "UniProtKB:Q32M45",
  "gene_symbol": "ANO4",
  "gene_name": "Anoctamin-4"
}